{
  "term_label": "postsynaptic density",
  "term_id": "GO:0014069",
  "gene_name": "Calcium_calmodulin-dependent protein kinase type II subunit delta",
  "gene_symbol": "CAMK2D",
  "gene": "UniProtKB:Q13557"
}